kanamycin biosynthetic process [GO:1901133] (biological process) Also known as: kanamycin anabolism, kanamycin biosynthesis, kanamycin formation, kanamycin synthesis Definition: The chemical reactions and pathways resulting in the formation of kanamycin. Relationships: is_a GO:0030648; is a type of polyol biosynthetic process [GO:0046173] Sources: GOC:TermGenie, GOC:yaf, UniPathway:UPA00965